phosphatidylinositol-3,5-bisphosphate phosphatase activity [GO:0106018] (molecular function) Definition: Catalysis of the reaction: 1-phosphatidyl-1D-myo-inositol 3,5-bisphosphate + H2O = 1-phosphatidyl-1D-myo-inositol phosphate + phosphate. Subtypes: phosphatidylinositol-3,5-bisphosphate 5-phosphatase activity [GO:0043813], phosphatidylinositol-3,5-bisphosphate 3-phosphatase activity [GO:0052629] Relationships: is a type of GO:0034593 Sources: GOC:hjd